{
  "gene_symbol": "CCL22",
  "gene_name": "C-C motif chemokine 22",
  "term_id": "GO:0005615",
  "gene": "UniProtKB:O00626",
  "term_label": "extracellular space"
}